{
  "gene": "UniProtKB:P0C879",
  "gene_symbol": "P0C879",
  "gene_name": "Putative uncharacterized protein FLJ43185",
  "term_label": "Unknown molecular function",
  "term_id": "UNKNOWN:0001"
}